protein-N(PI)-phosphohistidine-sugar phosphotransferase complex [GO:0009357] (cellular component) References: PMID:2951378 Relationships: is_a GO:0061695; is a type of GO:0140535; is a type of GO:1902495 Definition: An enzyme complex that catalyzes the transfer of a phosphate from protein N(PI)-phosphohistidine to a sugar molecule. It is enzyme II of the phosphotransferase system.